podosome assembly [GO:0071800] (biological process) Sources: GOC:mah, GOC:sl Definition: The aggregation, arrangement and bonding together of a set of components to form a podosome, an actin-rich adhesion structure characterized by formation upon cell substrate contact and localization at the substrate-attached part of the cell. Relationships: is a type of protein-containing complex assembly [GO:0065003]; is a type of membraneless organelle assembly [GO:0140694] Regulation: regulated by GO:0071801; negatively regulated by GO:0071802; positively regulated by GO:0071803